tetrahydroberberine oxidase activity [GO:0050328] (molecular function) Sources: EC:1.3.3.8, MetaCyc:TETRAHYDROBERBERINE-OXIDASE-RXN Definition: Catalysis of the reaction: (S)-tetrahydroberberine + 2 O2 = berberine + 2 H2O2. Also known as: (S)-THB oxidase activity, (S)-tetrahydroberberine:oxygen oxidoreductase activity, THB oxidase activity Relationships: is a type of GO:0016634